{
  "gene_name": "Protein lifeguard 2",
  "gene": "UniProtKB:Q9BWQ8",
  "term_label": "Golgi apparatus",
  "term_id": "GO:0005794",
  "gene_symbol": "FAIM2"
}